methylselenocysteine deselenhydrase activity [GO:0098607] (MF) Definition: Catalysis of the reaction: Se-Methyl-L-selenocysteine + H2O = pyruvic acid + NH3 + Methaneselenol. References: PMID:17451884, PMID:20383543 Relationships: is a type of carbon-sulfur lyase activity [GO:0016846]